{
  "gene_symbol": "DMAC2L",
  "term_id": "UNKNOWN:0001",
  "gene": "UniProtKB:Q99766",
  "gene_name": "ATP synthase subunit s, mitochondrial",
  "term_label": "Unknown molecular function"
}